interleukin-23 receptor binding [GO:0045519] (molecular function) Also known as: IL-23, interleukin-23 receptor ligand Relationships: is a type of cytokine receptor binding [GO:0005126] Sources: GOC:go_curators Definition: Binding to an interleukin-23 receptor.